{
  "gene_symbol": "GPRIN3",
  "gene": "UniProtKB:Q6ZVF9",
  "term_id": "GO:0005886",
  "term_label": "plasma membrane",
  "gene_name": "G protein-regulated inducer of neurite outgrowth 3"
}